beta-1 adrenergic receptor binding [GO:0031697] (molecular function) Also known as: beta-1 adrenergic receptor ligand Relationships: is_a GO:0031690 Definition: Binding to a beta-1 adrenergic receptor. Sources: GOC:mah, GOC:nln